{
  "gene_name": "Radial spoke head 1 homolog",
  "term_id": "GO:0005634",
  "gene_symbol": "RSPH1",
  "gene": "UniProtKB:Q8WYR4",
  "term_label": "nucleus"
}